nicotinamide mononucleotide transport [GO:0015890] (biological process) Subtypes: nicotinamide mononucleotide transmembrane transport [GO:0035353] Sources: ISBN:0721662544 Definition: The directed movement of nicotinamide mononucleotide into, out of or within a cell, or between cells, by means of some agent such as a transporter or pore. Nicotinamide mononucleotide is a ribonucleotide in which the nitrogenous base, nicotinamide, is in beta-n-glycosidic linkage with the c-1 position of D-ribose. It is a constituent of NAD and NADP. Relationships: is a type of nucleotide transport [GO:0006862]; is a type of carbohydrate derivative transport [GO:1901264] Also known as: nicotinamide ribonucleotide transport